microfibril assembly [GO:0160054] (biological process) Relationships: is a type of GO:0022607; is a type of GO:0097435 References: PMID:32855533 Definition: The aggregation, arrangement and bonding together of microfibril.